DNA-binding transcription factor activity [GO:0003700] (molecular function) Subtypes: DNA-binding transcription factor activity, RNA polymerase II-specific [GO:0000981], GO:0001216, DNA-binding transcription repressor activity [GO:0001217], sigma factor activity [GO:0016987], GO:0098531 Regulation: negatively regulated by negative regulation of DNA-binding transcription factor activity [GO:0043433]; regulated by regulation of DNA-binding transcription factor activity [GO:0051090]; positively regulated by GO:0051091 Also known as: nucleic acid binding transcription factor activity, transcription factor activity, DNA binding transcription factor activity, gene-specific transcription factor activity, sequence-specific DNA binding transcription factor activity, bacterial-type DNA binding transcription factor activity, bacterial-type RNA polymerase core promoter proximal region sequence-specific DNA binding transcription factor activity, bacterial-type RNA polymerase transcription enhancer sequence-specific DNA binding transcription factor activity, bacterial-type RNA polymerase transcription factor activity, metal ion regulated sequence-specific DNA binding, bacterial-type RNA polymerase transcription factor activity, sequence-specific DNA binding, metal ion regulated sequence-specific DNA binding bacterial-type RNA polymerase transcription factor activity, metal ion regulated sequence-specific DNA binding transcription factor activity, sequence-specific DNA binding bacterial-type RNA polymerase transcription factor activity, transcription factor activity, bacterial-type RNA polymerase core promoter proximal region sequence-specific binding, transcription factor activity, bacterial-type RNA polymerase proximal promoter sequence-specific DNA binding, transcription factor activity, bacterial-type RNA polymerase transcription enhancer sequence-specific binding, transcription factor activity, metal ion regulated sequence-specific DNA binding Sources: GOC:txnOH-2018 Relationships: is a type of transcription regulator activity [GO:0140110]; is part of regulation of DNA-templated transcription [GO:0006355]; has part transcription cis-regulatory region binding [GO:0000976] Note: Usage guidance: Most DNA-binding transcription factors do not have enzymatic activity. The presence of specific DNA-binding domains known to be present in DNA-binding transcription factors (HOX, GATA etc) should be used to help decide whether a protein is a DNA binding transcription factor or a coregulator. If a protein has an enzymatic activity (for example, ubiquitin ligase, histone acetyl transferase) and no known DNA binding domain, consider annotating to GO:0003712 transcription coregulator activity. Special care should be taken with proteins containing zinc fingers, Myb/SANT and ARID domains, since only a subset of proteins containing these domains directly and selectively bind to regulatory DNA motifs in cis-regulatory regions. Definition: A transcription regulator activity that modulates transcription of gene sets via selective and non-covalent binding to a specific double-stranded genomic DNA sequence (sometimes referred to as a motif) within a cis-regulatory region. Regulatory regions include promoters (proximal and distal) and enhancers. Genes are transcriptional units, and include bacterial operons.